response to insulin [GO:0032868] (biological process) Definition: Any process that results in a change in state or activity of a cell or an organism (in terms of movement, secretion, enzyme production, gene expression, etc.) as a result of an insulin stimulus. Insulin is a polypeptide hormone produced by the islets of Langerhans of the pancreas in mammals, and by the homologous organs of other organisms. Sources: GOC:mah, ISBN:0198506732 Also known as: response to insulin stimulus Relationships: is a type of response to peptide hormone [GO:0043434] Subtypes: cellular response to insulin stimulus [GO:0032869]